positive regulation of eye photoreceptor cell development [GO:0042479] (biological process) Definition: Any process that activates or increases the frequency, rate or extent of eye photoreceptor development. Relationships: is a type of GO:0010720; is a type of regulation of eye photoreceptor cell development [GO:0042478]; is a type of positive regulation of photoreceptor cell differentiation [GO:0046534]; positively regulates GO:0042462 Also known as: positive regulation of eye photoreceptor development, up regulation of eye photoreceptor cell development, up-regulation of eye photoreceptor cell development, upregulation of eye photoreceptor cell development, activation of eye photoreceptor cell development, stimulation of eye photoreceptor cell development Sources: GOC:jl Subtypes: positive regulation of compound eye photoreceptor development [GO:0045315]